negative regulation of supramolecular fiber organization [GO:1902904] (biological process) Definition: Any process that stops, prevents or reduces the frequency, rate or extent of fibril organization. Note: HSPA8, human, P11142 in PMID:23921388 inferred from direct assay to negatively regulate fibrillation of alpha-Syn in vitro Relationships: is a type of negative regulation of cellular component organization [GO:0051129]; is a type of regulation of supramolecular fiber organization [GO:1902903]; negatively regulates supramolecular fiber organization [GO:0097435] Subtypes: GO:0007026, negative regulation of actin filament depolymerization [GO:0030835], negative regulation of actin filament polymerization [GO:0030837], negative regulation of microtubule polymerization [GO:0031115], negative regulation of actin filament bundle assembly [GO:0032232], negative regulation of actin nucleation [GO:0051126], negative regulation of sarcomere organization [GO:0060299], negative regulation of myosin II filament organization [GO:1904900], GO:1905305, negative regulation of amyloid fibril formation [GO:1905907] Also known as: inhibition of fibril organisation, inhibition of fibril organization, down regulation of fibril organisation, down regulation of fibril organization, down-regulation of fibril organisation, down-regulation of fibril organization, downregulation of fibril organisation, downregulation of fibril organization, negative regulation of fibril organisation References: PMID:23921388 Sources: GOC:PARL, GOC:TermGenie, GOC:rl, GO_REF:0000058